{
  "gene_symbol": "NEO1",
  "gene": "UniProtKB:Q92859",
  "term_id": "UNKNOWN:0001",
  "term_label": "Unknown molecular function",
  "gene_name": "Neogenin"
}